{
  "gene_symbol": "PRELP",
  "gene_name": "Prolargin",
  "gene": "UniProtKB:P51888",
  "term_id": "GO:0008201",
  "term_label": "heparin binding"
}